{
  "gene_name": "Free fatty acid receptor 4",
  "gene": "UniProtKB:Q5NUL3",
  "term_id": "GO:0007186",
  "gene_symbol": "FFAR4",
  "term_label": "G protein-coupled receptor signaling pathway"
}